regulation of protein modification process [GO:0031399] (BP) Relationships: is a type of regulation of protein metabolic process [GO:0051246]; regulates protein modification process [GO:0036211] Subtypes: regulation of protein phosphorylation [GO:0001932], regulation of protein glutathionylation [GO:0010732], negative regulation of protein modification process [GO:0031400], positive regulation of protein modification process [GO:0031401], regulation of protein deacetylation [GO:0090311], GO:0120093, regulation of protein adenylylation [GO:1900722], GO:1901873, regulation of protein acetylation [GO:1901983], regulation of protein lipidation [GO:1903059], regulation of protein polyglycylation [GO:1903344], regulation of protein-pyridoxal-5-phosphate linkage [GO:1904285], regulation of protein oxidation [GO:1904806], regulation of peptidyl-cysteine S-nitrosylation [GO:2000169], regulation of protein geranylgeranylation [GO:2000539] Sources: GOC:mah, GOC:tb Definition: Any process that modulates the frequency, rate or extent of the covalent alteration of one or more amino acid residues within a protein.